oxidoreductase activity, acting on CH or CH2 groups, NAD or NADP as acceptor [GO:0016726] (molecular function) Sources: GOC:ai Subtypes: xanthine dehydrogenase activity [GO:0004854], leucoanthocyanidin reductase activity [GO:0033788], CDP-4-dehydro-6-deoxyglucose reductase activity [GO:0047099], nicotinate dehydrogenase activity [GO:0050138], GO:0070674 Definition: Catalysis of an oxidation-reduction (redox) reaction in which a CH2 group acts as a hydrogen or electron donor and reduces NAD+ or NADP. Relationships: is a type of oxidoreductase activity, acting on CH or CH2 groups [GO:0016725]